immune receptor activity [GO:0140375] (molecular function) Subtypes: complement receptor activity [GO:0004875], cytokine receptor activity [GO:0004896], GO:0019763, MHC class I receptor activity [GO:0032393], MHC class Ib receptor activity [GO:0032394], MHC class II receptor activity [GO:0032395], GO:0140376 Definition: Receiving a signal and transmitting it in a cell to initiate an immune response. Relationships: is a type of GO:0038023 References: PMID:31415752 Sources: Wikipedia:Immune_receptor